{
  "term_id": "GO:0005634",
  "gene_symbol": "PPP1CA",
  "gene": "UniProtKB:P62136",
  "gene_name": "Serine_threonine-protein phosphatase PP1-alpha catalytic subunit",
  "term_label": "nucleus"
}